{
  "term_label": "GTP binding",
  "gene": "UniProtKB:Q8IVW1",
  "term_id": "GO:0005525",
  "gene_name": "ADP-ribosylation factor-like protein 17",
  "gene_symbol": "ARL17A"
}